cortical actin cytoskeleton [GO:0030864] (cellular component) Subtypes: terminal web [GO:1990357] Sources: GOC:mah Relationships: is a type of cortical cytoskeleton [GO:0030863]; is part of actin cytoskeleton [GO:0015629] Definition: The portion of the actin cytoskeleton, comprising filamentous actin and associated proteins, that lies just beneath the plasma membrane.